{
  "gene": "UniProtKB:Q8WXI7",
  "term_id": "UNKNOWN:0003",
  "term_label": "Unknown cellular component",
  "gene_symbol": "MUC16",
  "gene_name": "Mucin-16"
}